{
  "gene_symbol": "NPY",
  "gene": "UniProtKB:P01303",
  "term_label": "extracellular space",
  "gene_name": "Pro-neuropeptide Y",
  "term_id": "GO:0005615"
}